{
  "term_label": "Unknown molecular function",
  "gene": "UniProtKB:A6NEH6",
  "gene_symbol": "TMEM247",
  "term_id": "UNKNOWN:0001",
  "gene_name": "Transmembrane protein 247"
}